{
  "gene_symbol": "DNAJA1",
  "gene": "UniProtKB:P31689",
  "term_id": "GO:0005829",
  "term_label": "cytosol",
  "gene_name": "DnaJ homolog subfamily A member 1"
}